formation of translation preinitiation complex [GO:0001731] (biological process) Definition: The joining of the small ribosomal subunit, ternary complex, and mRNA. Sources: GOC:hjd Also known as: formation of translation pre-initiation complex, translation preinitiation complex assembly Note: See also the cellular component terms 'eukaryotic 43S preinitiation complex ; GO:0016282', 'eukaryotic 48S initiation complex ; GO:0033290', and their children. Relationships: is a type of protein-RNA complex assembly [GO:0022618]; is part of GO:0002183 Regulation: regulated by regulation of formation of translation preinitiation complex [GO:1901193]; negatively regulated by GO:1901194; positively regulated by positive regulation of formation of translation preinitiation complex [GO:1901195]